{
  "term_id": "GO:0005615",
  "gene": "UniProtKB:P80108",
  "gene_symbol": "GPLD1",
  "term_label": "extracellular space",
  "gene_name": "Phosphatidylinositol-glycan-specific phospholipase D"
}